{
  "term_id": "GO:0007420",
  "gene": "UniProtKB:Q5SQQ9",
  "gene_name": "Ventral anterior homeobox 1",
  "gene_symbol": "VAX1",
  "term_label": "brain development"
}